{
  "term_label": "formation of cytoplasmic translation initiation complex",
  "gene_name": "Eukaryotic translation initiation factor 5",
  "term_id": "GO:0001732",
  "gene": "UniProtKB:P55010",
  "gene_symbol": "EIF5"
}